{
  "gene": "UniProtKB:Q9UI17",
  "gene_symbol": "DMGDH",
  "term_id": "UNKNOWN:0002",
  "term_label": "Unknown biological process",
  "gene_name": "Dimethylglycine dehydrogenase, mitochondrial"
}